negative regulation of autophagy [GO:0010507] (biological process) Subtypes: negative regulation of macroautophagy [GO:0016242], GO:1903147, negative regulation of chaperone-mediated autophagy [GO:1904715] Relationships: is a type of negative regulation of catabolic process [GO:0009895]; is a type of regulation of autophagy [GO:0010506]; negatively regulates GO:0006914 Definition: Any process that stops, prevents, or reduces the frequency, rate or extent of autophagy. Autophagy is the process in which cells digest parts of their own cytoplasm. Sources: GOC:dph, GOC:tb